{
  "gene": "UniProtKB:Q0VDD8",
  "term_label": "dynein intermediate chain binding",
  "gene_symbol": "DNAH14",
  "term_id": "GO:0045505",
  "gene_name": "Dynein axonemal heavy chain 14"
}